{
  "gene_name": "Putative PRAME family member 26",
  "gene": "UniProtKB:H0Y7S4",
  "term_id": "GO:1990756",
  "gene_symbol": "PRAMEF26",
  "term_label": "ubiquitin-like ligase-substrate adaptor activity"
}